{
  "gene": "UniProtKB:Q92753",
  "term_label": "melatonin receptor activity",
  "term_id": "GO:0008502",
  "gene_name": "Nuclear receptor ROR-beta",
  "gene_symbol": "RORB"
}